{
  "gene_name": "Spectrin beta chain, non-erythrocytic 5",
  "term_id": "GO:0030054",
  "gene_symbol": "SPTBN5",
  "gene": "UniProtKB:Q9NRC6",
  "term_label": "cell junction"
}